{
  "gene": "UniProtKB:P10244",
  "gene_name": "Myb-related protein B",
  "gene_symbol": "MYBL2",
  "term_label": "RNA polymerase II cis-regulatory region sequence-specific DNA binding",
  "term_id": "GO:0000978"
}